creatinine catabolic process to formate [GO:0019621] (biological process) Sources: GOC:go_curators Definition: The chemical reactions and pathways resulting in the breakdown of creatinine into other compounds, including formate. Relationships: is a type of creatinine catabolic process [GO:0006602]; is a type of formate metabolic process [GO:0015942] Also known as: creatinine breakdown to formate, creatinine degradation to formate